{
  "term_id": "GO:0000149",
  "gene_name": "Syntaxin-6",
  "gene_symbol": "STX6",
  "term_label": "SNARE binding",
  "gene": "UniProtKB:O43752"
}